axonemal heterotrimeric kinesin-II complex [GO:0030993] (cellular component) References: PMID:14570576 Sources: GOC:kmv Definition: A kinesin complex found in eukaryotic axonemes that contains two distinct plus end-directed kinesin motor proteins and at least one accessory subunit, and that functions in the anterograde transport of molecules (cargo) from the basal body to the distal tip of the axoneme. Relationships: is a type of GO:0032991; is part of axoneme [GO:0005930]